{
  "term_label": "Unknown cellular component",
  "gene_name": "Keratin-associated protein 7-1",
  "gene": "UniProtKB:Q8IUC3",
  "gene_symbol": "KRTAP7-1",
  "term_id": "UNKNOWN:0003"
}